peptidyl-threonine acetylation [GO:0120257] (biological process) Definition: The acetylation of peptidyl-threonine. References: PMID:16728640, PMID:22802624 Sources: GOC:krc Relationships: is a type of protein acetylation [GO:0006473] Subtypes: peptidyl-threonine O-acetylation [GO:0120258]